{
  "gene_name": "Ankyrin and armadillo repeat-containing protein",
  "term_label": "Unknown biological process",
  "term_id": "UNKNOWN:0002",
  "gene": "UniProtKB:Q7Z5J8",
  "gene_symbol": "ANKAR"
}